{
  "gene_symbol": "CTAGE6",
  "gene_name": "cTAGE family member 6",
  "term_label": "Unknown molecular function",
  "term_id": "UNKNOWN:0001",
  "gene": "UniProtKB:Q86UF2"
}